{
  "gene": "UniProtKB:Q8N319",
  "gene_symbol": "LINC03040",
  "term_label": "Unknown molecular function",
  "term_id": "UNKNOWN:0001",
  "gene_name": "Putative uncharacterized protein encoded by LINC03040"
}